ATP-dependent FeS chaperone activity [GO:0140663] (molecular function) Also known as: ATP-dependent FeS carrier activity References: PMID:16843540 Relationships: is a type of metallochaperone activity [GO:0016530]; is a type of ATP-dependent activity [GO:0140657] Definition: Binding to and delivering metal ions to a target protein, driven by ATP hydrolysis.